{
  "gene_name": "Hydroxymethylglutaryl-CoA synthase, mitochondrial",
  "term_label": "mitochondrion",
  "gene": "UniProtKB:P54868",
  "gene_symbol": "HMGCS2",
  "term_id": "GO:0005739"
}